{
  "gene": "UniProtKB:A6NIR3",
  "term_label": "GTPase activator activity",
  "term_id": "GO:0005096",
  "gene_name": "Arf-GAP with GTPase, ANK repeat and PH domain-containing protein 5",
  "gene_symbol": "AGAP5"
}